{
  "gene_symbol": "OPTN",
  "gene": "UniProtKB:Q96CV9",
  "term_label": "K63-linked polyubiquitin modification-dependent protein binding",
  "term_id": "GO:0070530",
  "gene_name": "Optineurin"
}